{
  "gene_symbol": "CYBB",
  "gene_name": "Cytochrome b-245 heavy chain",
  "term_label": "defense response",
  "term_id": "GO:0006952",
  "gene": "UniProtKB:P04839"
}